{
  "gene_symbol": "LRRC75B",
  "term_id": "UNKNOWN:0002",
  "gene": "UniProtKB:Q2VPJ9",
  "gene_name": "Leucine-rich repeat-containing protein 75B",
  "term_label": "Unknown biological process"
}